symbiont-mediated perturbation of host jasmonic acid signaling [GO:0052088] (biological process) Also known as: suppression by organism of host JA-mediated defense response, symbiont defense to host-produced jasmonic acid, activation by organism of defense-related host SA-mediated signal transduction pathway, activation by organism of defense-related host jasmonic acid-mediated signal transduction pathway, activation by symbiont of defense-related host jasmonic acid-mediated signal transduction pathway, down regulation by symbiont of host jasmonic acid-mediated defense response, down-regulation by symbiont of host jasmonic acid-mediated defense response, downregulation by symbiont of host jasmonic acid-mediated defense response, induction by organism of defense-related host SA-mediated signal transduction pathway, induction by organism of defense-related host jasmonic acid-mediated signal transduction pathway, induction by symbiont of defense-related host jasmonic acid-mediated signal transduction pathway, inhibition by symbiont of host jasmonic acid-mediated defense response, modulation by organism of defense-related jasmonic acid-mediated signal transduction pathway in other organism involved in symbiotic interaction, modulation by organism of host JA-mediated defense response, modulation by organism of jasmonic acid-mediated defense response of other organism involved in symbiotic interaction, modulation by symbiont of defense-related host jasmonic acid-mediated signal transduction pathway, negative regulation by organism of defense-related jasmonic acid-mediated signal transduction pathway in other organism involved in symbiotic interaction, negative regulation by organism of jasmonic acid-mediated defense response of other organism involved in symbiotic interaction, negative regulation by symbiont of defense-related host jasmonic acid-mediated signal transduction pathway, negative regulation by symbiont of host jasmonic acid-mediated defense response, positive regulation by organism of defense-related host SA-mediated signal transduction pathway, positive regulation by organism of defense-related jasmonic acid-mediated signal transduction pathway in other organism involved in symbiotic interaction, positive regulation by symbiont of defense-related host jasmonic acid-mediated signal transduction pathway, stimulation by symbiont of defense-related host jasmonic acid-mediated signal transduction pathway, up regulation by symbiont of defense-related host jasmonic acid-mediated signal transduction pathway, up-regulation by symbiont of defense-related host jasmonic acid-mediated signal transduction pathway, upregulation by organism of defense-related host SA-mediated signal transduction pathway, upregulation by organism of defense-related host jasmonic acid-mediated signal transduction pathway, upregulation by symbiont of defense-related host jasmonic acid-mediated signal transduction pathway, suppression by symbiont of host jasmonic acid-mediated defense response References: PMID:29222513, PMID:35698792 Sources: GOC:mtg_pamgo_17jul06 Relationships: is a type of GO:0052027; is a type of symbiont-mediated perturbation of host innate immune response [GO:0052167] Definition: A process in which a symbiont alters or subverts a jasmonic acid-mediated signal transduction pathway in its host. The host is defined as the larger of the organisms involved in a symbiotic interaction.